{
  "gene_symbol": "BICD2",
  "gene_name": "Protein bicaudal D homolog 2",
  "gene": "UniProtKB:Q8TD16",
  "term_label": "microtubule-based movement",
  "term_id": "GO:0007018"
}